co-receptor binding [GO:0039706] (molecular function) Definition: Binding to a coreceptor. A coreceptor acts in cooperation with a primary receptor to transmit a signal within the cell. Sources: GOC:bf, GOC:jl Relationships: is a type of protein binding [GO:0005515]